cellular response to codeine [GO:1905234] (biological process) Relationships: is a type of cellular response to isoquinoline alkaloid [GO:0071317]; is a type of GO:1905233 References: PMID:24914722 Sources: GOC:TermGenie, GO_REF:0000071 Definition: Any process that results in a change in state or activity of a cell (in terms of movement, secretion, enzyme production, gene expression, etc.) as a result of a codeine stimulus.